methylammonium transport [GO:0015843] (biological process) Subtypes: methylammonium transmembrane transport [GO:0072489] Sources: GOC:ai Relationships: is a type of organic cation transport [GO:0015695]; is a type of GO:0015837; is a type of one-carbon compound transport [GO:0019755] Definition: The directed movement of methylammonium into, out of or within a cell, or between cells, by means of some agent such as a transporter or pore.